{
  "term_label": "angiogenesis",
  "gene_name": "Calcitonin gene-related peptide type 1 receptor",
  "gene_symbol": "CALCRL",
  "term_id": "GO:0001525",
  "gene": "UniProtKB:Q16602"
}